{
  "gene_symbol": "MCOLN3",
  "term_id": "GO:0005886",
  "gene_name": "Mucolipin-3",
  "gene": "UniProtKB:Q8TDD5",
  "term_label": "plasma membrane"
}